segment specification [GO:0007379] (biological process) Relationships: is_a GO:0007389; is part of GO:0035282 Definition: The process in which segments assume individual identities; exemplified in insects by the actions of the products of the homeotic genes. Subtypes: somite specification [GO:0001757], specification of segmental identity, head [GO:0007380], specification of segmental identity, trunk [GO:0035292], specification of nephron tubule identity [GO:0072081] Sources: ISBN:0879694238, http://fly.ebi.ac.uk/allied-data/lk/interactive-fly/aimain/1aahome.htm